{
  "term_label": "cellular response to oxidative stress",
  "term_id": "GO:0034599",
  "gene_name": "Phospholipid hydroperoxide glutathione peroxidase",
  "gene_symbol": "GPX4",
  "gene": "UniProtKB:P36969"
}